positive regulation of sterol transport [GO:0032373] (biological process) Sources: GOC:mah Relationships: is a type of positive regulation of lipid transport [GO:0032370]; is a type of regulation of sterol transport [GO:0032371]; positively regulates GO:0015918 Subtypes: positive regulation of cholesterol transport [GO:0032376], GO:0032382, positive regulation of sterol import [GO:2000911] Also known as: up regulation of sterol transport, up-regulation of sterol transport, upregulation of sterol transport, activation of sterol transport, stimulation of sterol transport Definition: Any process that activates or increases the frequency, rate or extent of the directed movement of sterols into, out of or within a cell, or between cells, by means of some agent such as a transporter or pore.